{
  "gene": "UniProtKB:Q9NQ87",
  "gene_symbol": "HEYL",
  "term_id": "GO:0007219",
  "term_label": "Notch signaling pathway",
  "gene_name": "Hairy_enhancer-of-split related with YRPW motif-like protein"
}